{
  "gene_symbol": "DEFB109B",
  "gene": "UniProtKB:Q30KR1",
  "term_label": "chemoattractant activity",
  "gene_name": "Putative beta-defensin 109B",
  "term_id": "GO:0042056"
}